{
  "gene_symbol": "C10orf62",
  "term_id": "UNKNOWN:0002",
  "gene": "UniProtKB:Q5T681",
  "gene_name": "Uncharacterized protein C10orf62",
  "term_label": "Unknown biological process"
}